leukocyte degranulation [GO:0043299] (biological process) Regulation: regulated by GO:0043300; negatively regulated by negative regulation of leukocyte degranulation [GO:0043301]; positively regulated by positive regulation of leukocyte degranulation [GO:0043302] Subtypes: basophil degranulation [GO:0002561], mast cell degranulation [GO:0043303], eosinophil degranulation [GO:0043308], neutrophil degranulation [GO:0043312], GO:0043316, natural killer cell degranulation [GO:0043320] Definition: The regulated exocytosis of secretory granules by a leukocyte. Sources: GOC:add, GO_REF:0000022, ISBN:0781735149 Also known as: immune cell degranulation, immune cell granule exocytosis, leucocyte degranulation, leukocyte granule exocytosis Relationships: is a type of immune effector process [GO:0002252]; is_a GO:0045055; is a type of establishment of localization in cell [GO:0051649]